proteasome accessory complex [GO:0022624] (cellular component) Sources: GOC:mtg_sensu Definition: A protein complex, that caps one or both ends of the proteasome core complex and regulates entry into, or exit from, the proteasome core complex. Relationships: is_a protein-containing complex [GO:0032991]; is part of proteasome complex [GO:0000502]; is part of intracellular anatomical structure [GO:0005622]